{
  "term_id": "GO:0043536",
  "gene_symbol": "AKT1",
  "term_label": "positive regulation of blood vessel endothelial cell migration",
  "gene_name": "RAC-alpha serine_threonine-protein kinase",
  "gene": "UniProtKB:P31749"
}